{
  "gene_symbol": "CLDN15",
  "gene": "UniProtKB:P56746",
  "term_label": "bicellular tight junction",
  "gene_name": "Claudin-15",
  "term_id": "GO:0005923"
}